neurotransmitter receptor transport, endosome to plasma membrane [GO:0099639] (biological process) Subtypes: GO:0098887 Relationships: is a type of neurotransmitter receptor transport to plasma membrane [GO:0098877]; is a type of endosome to plasma membrane protein transport [GO:0099638] Definition: The directed movement of neurotransmitter receptor from the endosome to the plasma membrane in transport vesicles. Sources: GOC:dos